{
  "gene_name": "Protein AF-17",
  "gene": "UniProtKB:P55198",
  "term_label": "histone reader activity",
  "term_id": "GO:0140566",
  "gene_symbol": "MLLT6"
}